{
  "gene_symbol": "MYL6",
  "term_label": "microfilament motor activity",
  "term_id": "GO:0000146",
  "gene_name": "Myosin light polypeptide 6",
  "gene": "UniProtKB:P60660"
}